{
  "term_label": "smoothened signaling pathway",
  "gene_name": "SCL-interrupting locus protein",
  "gene_symbol": "STIL",
  "gene": "UniProtKB:Q15468",
  "term_id": "GO:0007224"
}